{
  "gene_symbol": "SCG2",
  "term_label": "eosinophil chemotaxis",
  "gene": "UniProtKB:P13521",
  "gene_name": "Secretogranin-2",
  "term_id": "GO:0048245"
}